{
  "gene_name": "Dynein heavy chain domain-containing protein 1",
  "term_id": "GO:0030317",
  "gene": "UniProtKB:Q96M86",
  "gene_symbol": "DNHD1",
  "term_label": "flagellated sperm motility"
}